{
  "term_label": "regulation of stem cell population maintenance",
  "gene": "UniProtKB:Q9NZN8",
  "gene_name": "CCR4-NOT transcription complex subunit 2",
  "gene_symbol": "CNOT2",
  "term_id": "GO:2000036"
}